heterochromatin island [GO:1990342] (cellular component) Relationships: is a type of heterochromatin [GO:0000792] Note: An example of this type of heterochromatin is found in Schizosaccharomyces pombe, where heterochromatin islands are formed at meiotic genes during vegetative (mitotic) growth. References: PMID:22144463, PMID:24210919 Definition: A region of facultative heterochromatin formed dynamically at specific loci in response to environmental signals, independently of RNAi.